{
  "term_label": "cytoplasm",
  "term_id": "GO:0005737",
  "gene": "UniProtKB:P01036",
  "gene_symbol": "CST4",
  "gene_name": "Cystatin-S"
}